{
  "gene_symbol": "TRRAP",
  "term_label": "SAGA complex",
  "gene_name": "Transformation_transcription domain-associated protein",
  "term_id": "GO:0000124",
  "gene": "UniProtKB:Q9Y4A5"
}